mRNA (cytidine-5-)-methyltransferase activity [GO:0062152] (molecular function) References: PMID:22395603, PMID:23871666 Sources: RHEA:61464 Definition: Catalysis of the reaction: a cytidine in mRNA + S-adenosyl-L-methionine = a 5-methylcytidine in mRNA + H+ + S-adenosyl-L-homocysteine. Relationships: is a type of mRNA methyltransferase activity [GO:0008174] Also known as: mRNA (cytosine-5-)-methyltransferase activity